{
  "term_label": "four-way junction helicase activity",
  "gene": "UniProtKB:P54132",
  "gene_symbol": "BLM",
  "term_id": "GO:0009378",
  "gene_name": "RecQ-like DNA helicase BLM"
}